{
  "term_id": "GO:0045454",
  "gene_symbol": "KRIT1",
  "term_label": "cell redox homeostasis",
  "gene": "UniProtKB:O00522",
  "gene_name": "Krev interaction trapped protein 1"
}